tricarboxylic acid cycle heteromeric enzyme complex [GO:0045239] (CC) Relationships: is a type of catalytic complex [GO:1902494]; is part of cytoplasm [GO:0005737] Also known as: TCA cycle enzyme complex Subtypes: succinate-CoA ligase complex [GO:0042709], isocitrate dehydrogenase complex (NAD+) [GO:0045242], oxoglutarate dehydrogenase complex [GO:0045252] Definition: Any of the heteromeric enzymes that act in the TCA cycle. Sources: GOC:mah